{
  "term_label": "cellular response to light stimulus",
  "gene_name": "Medium-wave-sensitive opsin 1",
  "gene_symbol": "OPN1MW",
  "term_id": "GO:0071482",
  "gene": "UniProtKB:P04001"
}